{
  "gene_name": "Vitamin K-dependent protein Z",
  "gene": "UniProtKB:P22891",
  "term_id": "GO:0004252",
  "gene_symbol": "PROZ",
  "term_label": "serine-type endopeptidase activity"
}